{
  "gene_name": "Keratin, type I cuticular Ha7",
  "gene": "UniProtKB:O76014",
  "gene_symbol": "KRT37",
  "term_label": "structural constituent of skin epidermis",
  "term_id": "GO:0030280"
}